{
  "gene": "UniProtKB:Q04656",
  "gene_symbol": "ATP7A",
  "term_id": "GO:0060003",
  "gene_name": "Copper-transporting ATPase 1",
  "term_label": "copper ion export"
}